{
  "term_id": "GO:0005886",
  "term_label": "plasma membrane",
  "gene": "UniProtKB:Q50LG9",
  "gene_name": "Leucine-rich repeat-containing protein 24",
  "gene_symbol": "LRRC24"
}